{
  "gene": "UniProtKB:Q0VAK6",
  "gene_name": "Leiomodin-3",
  "term_id": "GO:0030239",
  "gene_symbol": "LMOD3",
  "term_label": "myofibril assembly"
}